{
  "gene_name": "Cerebellin-2",
  "term_label": "maintenance of synapse structure",
  "gene_symbol": "CBLN2",
  "gene": "UniProtKB:Q8IUK8",
  "term_id": "GO:0099558"
}